{
  "term_id": "GO:0008284",
  "gene_name": "Homeobox protein Meis1",
  "term_label": "positive regulation of cell population proliferation",
  "gene_symbol": "MEIS1",
  "gene": "UniProtKB:O00470"
}